UTP:glucose-1-phosphate uridylyltransferase activity [GO:0003983] (molecular function) Relationships: is a type of UTP-monosaccharide-1-phosphate uridylyltransferase activity [GO:0051748] Definition: Catalysis of the reaction: alpha-D-glucose 1-phosphate + UTP = diphosphate + UDP-D-glucose. Also known as: UDP glucose pyrophosphorylase activity, UDP-glucose diphosphorylase activity, UDP-glucose pyrophosphorylase activity, UDPG phosphorylase activity, UDPG pyrophosphorylase activity, UTP-glucose-1-phosphate uridylyltransferase activity, UTP:alpha-D-glucose-1-phosphate uridylyltransferase activity, glucose-1-phosphate uridylyltransferase activity, uridine 5'-diphosphoglucose pyrophosphorylase activity, uridine diphosphate-D-glucose pyrophosphorylase activity, uridine diphosphoglucose pyrophosphorylase activity, uridine-diphosphate glucose pyrophosphorylase activity Sources: EC:2.7.7.9, RHEA:19889 Regulation: regulated by UTP:glucose-1-phosphate uridylyltransferase regulator activity [GO:0043763]